L-kynurenine transmembrane transport [GO:0140924] (biological process) Definition: The directed movement of L-kynurenine across a membrane. Relationships: is a type of GO:1902475 References: PMID:35245456